23S rRNA (guanine(1835)-N(2))-methyltransferase activity [GO:0052916] (molecular function) Definition: Catalysis of the reaction: S-adenosyl-L-methionine + guanosine(1835) in 23S rRNA = N(2)-methylguanosine(1835) in 23S rRNA + S-adenosyl-L-homocysteine. Relationships: is a type of rRNA (guanine-N2-)-methyltransferase activity [GO:0008990] Sources: EC:2.1.1.174